{
  "gene_name": "Receptor-type tyrosine-protein phosphatase O",
  "term_id": "GO:0098982",
  "gene": "UniProtKB:Q16827",
  "gene_symbol": "PTPRO",
  "term_label": "GABA-ergic synapse"
}